cell adhesive protein binding involved in atrial cardiac muscle cell-AV node cell communication [GO:0086081] (molecular function) Sources: GOC:BHF, GOC:mtg_cardiac_conduct_nov11 Relationships: is a type of protein binding involved in heterotypic cell-cell adhesion [GO:0086080]; is part of atrial cardiac muscle cell-AV node cell adhesion involved in cell communication [GO:0086071] Also known as: cell adhesive protein binding involved in atrial cardiomyocyte-AV node cell communication, cell adhesive protein binding involved in atrial cardiomyocyte-atrioventricular node cell communication Definition: Binding to a protein or protein complex that results in the connection of an atrial cardiomyocyte with an AV node cell and contributes to the communication between the two cells.